negative regulation of cardiac muscle contraction [GO:0055118] (BP) Definition: Any process that stops, prevents, or reduces the frequency, rate or extent of cardiac muscle contraction. Sources: GOC:ecd Subtypes: negative regulation of cardiac muscle cell contraction [GO:0106135] Relationships: is a type of negative regulation of heart contraction [GO:0045822]; is a type of GO:0045988; is a type of regulation of cardiac muscle contraction [GO:0055117]; negatively regulates cardiac muscle contraction [GO:0060048]